lipoprotein oxidation [GO:0042161] (biological process) Definition: The modification of a lipoprotein by oxidation of one or more amino acids or the lipid group. Sources: GOC:mah Relationships: is a type of GO:0042160 Subtypes: lipoprotein lipid oxidation [GO:0034439] Regulation: regulated by regulation of lipoprotein oxidation [GO:0034442]; negatively regulated by negative regulation of lipoprotein oxidation [GO:0034443]